{
  "gene_symbol": "ZNF131",
  "gene_name": "Zinc finger protein 131",
  "term_id": "GO:0000122",
  "gene": "UniProtKB:P52739",
  "term_label": "negative regulation of transcription by RNA polymerase II"
}